siRNA-mediated gene silencing by inhibition of translation [GO:0070549] (biological process) Relationships: is a type of negative regulation of translation [GO:0017148]; is a type of siRNA-mediated post-transcriptional gene silencing [GO:0140766] Definition: An siRNA-mediated post-transcriptional gene silencing pathway that blocks the translation of target mRNAs into proteins. Once incorporated into a RNA-induced silencing complex (RISC), an siRNA will typically mediate repression of translation if the siRNA perfectly complements elements located in the 3' untranslated region of target mRNAs. References: PMID:18771919 Sources: GOC:mah Also known as: down regulation of translation involved in RNA interference, down-regulation of translation involved in RNA interference, downregulation of translation involved in RNA interference, inhibition of translation involved in RNA interference, negative regulation of translation involved in RNA interference, RNA interference, negative regulation of translation